{
  "gene_symbol": "AP2A1",
  "term_label": "AP-2 adaptor complex",
  "gene_name": "AP-2 complex subunit alpha-1",
  "term_id": "GO:0030122",
  "gene": "UniProtKB:O95782"
}